{
  "gene": "UniProtKB:P0C7Q2",
  "gene_symbol": "ARMS2",
  "term_label": "Unknown molecular function",
  "gene_name": "Age-related maculopathy susceptibility protein 2",
  "term_id": "UNKNOWN:0001"
}